regulation of catalytic activity [GO:0050790] (biological process) Subtypes: GO:0032071, positive regulation of catalytic activity [GO:0043085], negative regulation of catalytic activity [GO:0043086], regulation of adenylate cyclase activity [GO:0045761], GO:0051336, regulation of transferase activity [GO:0051338], GO:0051341, regulation of ribonuclease activity [GO:0060700], regulation of deacetylase activity [GO:0150065], regulation of tocopherol cyclase activity [GO:1902171], regulation of RNA helicase activity [GO:1902280] Also known as: regulation of enzyme activity, regulation of metalloenzyme activity Definition: Any process that modulates the activity of an enzyme. Relationships: is a type of GO:0065009; regulates GO:0003824 Sources: GOC:ai, GOC:ebc, GOC:vw